{
  "gene_symbol": "BCL6B",
  "term_id": "GO:0001817",
  "gene": "UniProtKB:Q8N143",
  "term_label": "regulation of cytokine production",
  "gene_name": "B-cell CLL_lymphoma 6 member B protein"
}